{
  "term_label": "phosphatidylserine exposure on apoptotic cell surface",
  "term_id": "GO:0070782",
  "gene": "UniProtKB:Q9H6D3",
  "gene_symbol": "XKR8",
  "gene_name": "XK-related protein 8"
}